{
  "gene_symbol": "ZNF528",
  "term_id": "GO:0000981",
  "gene_name": "Zinc finger protein 528",
  "term_label": "DNA-binding transcription factor activity, RNA polymerase II-specific",
  "gene": "UniProtKB:Q3MIS6"
}